{
  "gene_symbol": "MED30",
  "term_id": "GO:0003712",
  "term_label": "transcription coregulator activity",
  "gene_name": "Mediator of RNA polymerase II transcription subunit 30",
  "gene": "UniProtKB:Q96HR3"
}